{
  "term_label": "plasma membrane",
  "gene": "UniProtKB:Q7L1W4",
  "gene_symbol": "LRRC8D",
  "gene_name": "Volume-regulated anion channel subunit LRRC8D",
  "term_id": "GO:0005886"
}